{
  "gene_name": "Chromodomain-helicase-DNA-binding protein 5",
  "term_label": "histone binding",
  "gene_symbol": "CHD5",
  "term_id": "GO:0042393",
  "gene": "UniProtKB:Q8TDI0"
}